{
  "gene_symbol": "NOX1",
  "term_label": "NAD(P)H oxidase H2O2-forming activity",
  "gene": "UniProtKB:Q9Y5S8",
  "gene_name": "NADPH oxidase 1",
  "term_id": "GO:0016174"
}